{
  "term_id": "GO:0003333",
  "gene_symbol": "SLC7A6",
  "term_label": "amino acid transmembrane transport",
  "gene": "UniProtKB:Q92536",
  "gene_name": "Y+L amino acid transporter 2"
}